{
  "term_label": "signal transduction",
  "term_id": "GO:0007165",
  "gene_symbol": "OR1E3",
  "gene_name": "Olfactory receptor 1E3",
  "gene": "UniProtKB:Q8WZA6"
}